{
  "gene_symbol": "CARD11",
  "term_id": "GO:0005886",
  "term_label": "plasma membrane",
  "gene_name": "Caspase recruitment domain-containing protein 11",
  "gene": "UniProtKB:Q9BXL7"
}